{
  "gene_symbol": "PIP4K2A",
  "term_id": "GO:0016309",
  "term_label": "1-phosphatidylinositol-5-phosphate 4-kinase activity",
  "gene": "UniProtKB:P48426",
  "gene_name": "Phosphatidylinositol 5-phosphate 4-kinase type-2 alpha"
}